{
  "term_label": "regulation of mitochondrial membrane permeability involved in programmed necrotic cell death",
  "gene_symbol": "PPIF",
  "gene_name": "Peptidyl-prolyl cis-trans isomerase F, mitochondrial",
  "gene": "UniProtKB:P30405",
  "term_id": "GO:1902445"
}